{
  "term_label": "regulation of inflammatory response",
  "gene": "UniProtKB:Q9NX02",
  "term_id": "GO:0050727",
  "gene_name": "NACHT, LRR and PYD domains-containing protein 2",
  "gene_symbol": "NLRP2"
}